{
  "term_id": "GO:0016491",
  "gene": "UniProtKB:P00450",
  "gene_symbol": "CP",
  "gene_name": "Ceruloplasmin",
  "term_label": "oxidoreductase activity"
}